{
  "term_label": "positive regulation of cell population proliferation",
  "gene_symbol": "FGF6",
  "term_id": "GO:0008284",
  "gene_name": "Fibroblast growth factor 6",
  "gene": "UniProtKB:P10767"
}